positive regulation of ribosomal large subunit export from nucleus [GO:2000205] (biological process) Definition: Any process that activates or increases the frequency, rate or extent of ribosomal large subunit export from nucleus. Sources: GOC:mah Also known as: positive regulation of ribosomal large subunit export from cell nucleus, positive regulation of ribosomal large subunit export out of nucleus, positive regulation of ribosomal large subunit transport from nucleus to cytoplasm, positive regulation of ribosomal large subunit-nucleus export, positive regulation of 50S ribosomal subunit export from nucleus, positive regulation of 60S ribosomal subunit export from nucleus Relationships: is a type of positive regulation of ribosomal subunit export from nucleus [GO:2000202]; is a type of regulation of ribosomal large subunit export from nucleus [GO:2000203]; positively regulates GO:0000055